symbiont-containing vacuolar space [GO:0020004] (cellular component) Relationships: is a type of membrane-enclosed lumen [GO:0031974]; BFO_0000050 symbiont-containing vacuole [GO:0020003] Definition: The space between a symbiont plasma membrane and the symbiont-containing vacuole membrane. Sources: GOC:jl, GOC:mb Also known as: parasitophorous vacuolar space, symbiont-containing vacuole space